{
  "term_id": "GO:0005634",
  "gene_symbol": "FBXL21P",
  "gene_name": "Putative F-box_LRR-repeat protein 21",
  "gene": "UniProtKB:Q9UKT6",
  "term_label": "nucleus"
}